{
  "gene": "UniProtKB:Q4FZB7",
  "term_label": "Unknown biological process",
  "gene_symbol": "KMT5B",
  "gene_name": "Histone-lysine N-methyltransferase KMT5B",
  "term_id": "UNKNOWN:0002"
}